{
  "term_id": "GO:0005886",
  "gene_name": "Synaptosomal-associated protein 47",
  "term_label": "plasma membrane",
  "gene_symbol": "SNAP47",
  "gene": "UniProtKB:Q5SQN1"
}